{
  "term_id": "GO:0005689",
  "gene_name": "RNA-binding protein 41",
  "gene_symbol": "RBM41",
  "term_label": "U12-type spliceosomal complex",
  "gene": "UniProtKB:Q96IZ5"
}